{
  "gene_symbol": "XYLT1",
  "term_id": "UNKNOWN:0003",
  "term_label": "Unknown cellular component",
  "gene": "UniProtKB:Q86Y38",
  "gene_name": "Xylosyltransferase 1"
}